{
  "gene": "UniProtKB:P26951",
  "gene_symbol": "IL3RA",
  "term_label": "external side of plasma membrane",
  "term_id": "GO:0009897",
  "gene_name": "Interleukin-3 receptor subunit alpha"
}